CCR3 chemokine receptor binding [GO:0031728] (molecular function) Relationships: is a type of GO:0048020 Also known as: eosinophil eotaxin receptor binding, CCR3 chemokine receptor ligand Sources: GOC:mah, GOC:nln Definition: Binding to a CCR3 chemokine receptor.